{
  "term_label": "RNA binding",
  "gene_symbol": "RAE1",
  "gene_name": "mRNA export factor RAE1",
  "gene": "UniProtKB:P78406",
  "term_id": "GO:0003723"
}